{
  "gene": "UniProtKB:P12272",
  "term_label": "hormone activity",
  "gene_name": "Parathyroid hormone-related protein",
  "term_id": "GO:0005179",
  "gene_symbol": "PTHLH"
}